{
  "term_id": "UNKNOWN:0003",
  "gene": "UniProtKB:P59827",
  "gene_name": "BPI fold-containing family B member 4",
  "gene_symbol": "BPIFB4",
  "term_label": "Unknown cellular component"
}